{
  "gene": "UniProtKB:Q92887",
  "term_id": "GO:0055085",
  "gene_symbol": "ABCC2",
  "term_label": "transmembrane transport",
  "gene_name": "ATP-binding cassette sub-family C member 2"
}